{
  "term_label": "membrane",
  "term_id": "GO:0016020",
  "gene": "UniProtKB:Q6ZMI0",
  "gene_name": "Protein phosphatase 1 regulatory subunit 21",
  "gene_symbol": "PPP1R21"
}